{
  "term_label": "Unknown molecular function",
  "gene_symbol": "C9orf40",
  "term_id": "UNKNOWN:0001",
  "gene": "UniProtKB:Q8IXQ3",
  "gene_name": "Uncharacterized protein C9orf40"
}